{
  "gene_symbol": "CHD4",
  "term_label": "ATP hydrolysis activity",
  "gene": "UniProtKB:Q14839",
  "gene_name": "Chromodomain-helicase-DNA-binding protein 4",
  "term_id": "GO:0016887"
}